{
  "gene_symbol": "MASP2",
  "gene_name": "Mannan-binding lectin serine protease 2",
  "term_label": "extracellular space",
  "gene": "UniProtKB:O00187",
  "term_id": "GO:0005615"
}